{
  "gene_name": "Putative postmeiotic segregation increased 2-like protein 3",
  "gene_symbol": "PMS2P3",
  "gene": "UniProtKB:Q13401",
  "term_id": "UNKNOWN:0002",
  "term_label": "Unknown biological process"
}